{
  "gene_name": "Zinc finger protein ubi-d4",
  "gene_symbol": "DPF2",
  "term_label": "negative regulation of myeloid progenitor cell differentiation",
  "term_id": "GO:1905454",
  "gene": "UniProtKB:Q92785"
}